{
  "term_id": "UNKNOWN:0001",
  "gene_name": "Cornifin-B",
  "term_label": "Unknown molecular function",
  "gene_symbol": "SPRR1B",
  "gene": "UniProtKB:P22528"
}